{
  "term_label": "Unknown cellular component",
  "term_id": "UNKNOWN:0003",
  "gene": "UniProtKB:A0A6Q8PHR7",
  "gene_symbol": "A0A6Q8PHR7",
  "gene_name": "Uncharacterized protein"
}